{
  "gene_name": "Killer cell immunoglobulin-like receptor 3DL2",
  "gene": "UniProtKB:P43630",
  "term_id": "GO:0002767",
  "gene_symbol": "KIR3DL2",
  "term_label": "immune response-inhibiting cell surface receptor signaling pathway"
}